glutaminyl-tRNA aminoacylation [GO:0006425] (biological process) Definition: The process of coupling glutamine to glutaminyl-tRNA, catalyzed by glutaminyl-tRNA synthetase. The glutaminyl-tRNA synthetase is a class-I synthetase. The activated amino acid is transferred to the 2'-OH group of a glutamine-accetping tRNA. The 2'-O-aminoacyl-tRNA will ultimately migrate to the 3' position via transesterification. Subtypes: mitochondrial glutaminyl-tRNA aminoacylation [GO:0070148] Sources: GOC:mcc, ISBN:0716730510 Relationships: is a type of tRNA aminoacylation for protein translation [GO:0006418]